{
  "gene": "UniProtKB:Q53H47",
  "gene_name": "Histone-lysine N-methyltransferase SETMAR",
  "term_label": "double-strand break repair via nonhomologous end joining",
  "gene_symbol": "SETMAR",
  "term_id": "GO:0006303"
}